positive regulation of DNA biosynthetic process [GO:2000573] (biological process) Sources: GOC:obol Subtypes: positive regulation of telomere maintenance via telomerase [GO:0032212], positive regulation of DNA-directed DNA polymerase activity [GO:1900264], positive regulation of reverse transcription [GO:1900270], GO:1904333, GO:1904525 Also known as: positive regulation of DNA anabolism, positive regulation of DNA biosynthesis, positive regulation of DNA formation, positive regulation of DNA synthesis Relationships: is a type of positive regulation of macromolecule biosynthetic process [GO:0010557]; is_a positive regulation of DNA metabolic process [GO:0051054]; is_a regulation of DNA biosynthetic process [GO:2000278]; positively regulates GO:0071897 Definition: Any process that activates or increases the frequency, rate or extent of DNA biosynthetic process.